{
  "gene_symbol": "PAK3",
  "term_id": "GO:0009267",
  "term_label": "cellular response to starvation",
  "gene_name": "Serine_threonine-protein kinase PAK 3",
  "gene": "UniProtKB:O75914"
}